{
  "gene_name": "Rabphilin-3A",
  "term_id": "GO:0045202",
  "gene": "UniProtKB:Q9Y2J0",
  "gene_symbol": "RPH3A",
  "term_label": "synapse"
}